{
  "gene_symbol": "POLR2L",
  "term_label": "RNA polymerase I complex",
  "gene": "UniProtKB:P62875",
  "gene_name": "DNA-directed RNA polymerases I, II, and III subunit RPABC5",
  "term_id": "GO:0005736"
}